adenylylselenate kinase activity [GO:0098617] (molecular function) Relationships: is a type of GO:0016773 References: PMID:2537056 Definition: Catalysis of the reaction: ATP + adenylylselenate = ADP + 3'-phosphoadenylylselenate.